modulation of inhibitory postsynaptic potential [GO:0098828] (biological process) Also known as: regulation of inhibitory postsynaptic potential Subtypes: positive regulation of inhibitory postsynaptic potential [GO:0097151] Relationships: is a type of regulation of signal transduction [GO:0009966]; is a type of regulation of nervous system process [GO:0031644]; is_a GO:0042391; regulates inhibitory postsynaptic potential [GO:0060080] Sources: GOC:dos Definition: Any process that modulates the frequency, rate or extent of inhibitory postsynaptic potential (IPSP). IPSP is a temporary decrease in postsynaptic membrane potential due to the flow of negatively charged ions into the postsynaptic cell. The flow of ions that causes an IPSP is an inhibitory postsynaptic current (IPSC) and makes it more difficult for the neuron to fire an action potential.